{
  "term_label": "Unknown cellular component",
  "term_id": "UNKNOWN:0003",
  "gene_name": "Endogenous retrovirus group K member 10 Pol protein",
  "gene": "UniProtKB:P10266",
  "gene_symbol": "ERVK-10"
}